{
  "gene": "UniProtKB:A8MV65",
  "term_id": "GO:0006357",
  "term_label": "regulation of transcription by RNA polymerase II",
  "gene_name": "Transcription cofactor vestigial-like protein 3",
  "gene_symbol": "VGLL3"
}